{
  "gene_name": "Regulator of MON1-CCZ1 complex",
  "gene": "UniProtKB:Q96DM3",
  "gene_symbol": "RMC1",
  "term_id": "GO:0010506",
  "term_label": "regulation of autophagy"
}